{
  "gene_name": "Neuron-specific vesicular protein calcyon",
  "term_label": "endosome",
  "gene": "UniProtKB:Q9NYX4",
  "term_id": "GO:0005768",
  "gene_symbol": "CALY"
}